extracellular matrix structural constituent conferring compression resistance [GO:0030021] (molecular function) Definition: A constituent of the extracellular matrix that enables the matrix to resist compressive forces; often a proteoglycan. Sources: GOC:mah, ISBN:0815316194 Also known as: core extracellular matrix, core matrisome Note: Extracellular matrix proteoglycans may be annotated to this term. PMID:8346704 Relationships: is a type of extracellular matrix structural constituent [GO:0005201] Subtypes: structural constituent of tooth enamel [GO:0030345]